{
  "gene": "UniProtKB:P17152",
  "gene_name": "Transmembrane protein 11, mitochondrial",
  "term_label": "Unknown molecular function",
  "term_id": "UNKNOWN:0001",
  "gene_symbol": "TMEM11"
}